mast cell granule [GO:0042629] (cellular component) Definition: Coarse, bluish-black staining cytoplasmic granules, bounded by a plasma membrane and found in mast cells and basophils. Contents include histamine, heparin, chondroitin sulfates, chymase and tryptase. References: PMID:12360215 Sources: GOC:jl Relationships: is a type of lysosome [GO:0005764]